{
  "gene_name": "Probable G-protein coupled receptor 149",
  "term_label": "neuropeptide signaling pathway",
  "gene_symbol": "GPR149",
  "term_id": "GO:0007218",
  "gene": "UniProtKB:Q86SP6"
}